lipid A-core heptosyltransferase activity [GO:0071968] (molecular function) Definition: Catalysis of the reaction: galactosyl-glucosyl3-heptosyl3-KDO2-lipid A-bisphosphate + ADP-L-glycero-beta-D-manno-heptose = lipid A-core + ADP + H+. Sources: MetaCyc:RXN0-5127 Relationships: is a type of lipopolysaccharide heptosyltransferase activity [GO:0008920]